regulation of substance P secretion [GO:1904458] (biological process) References: PMID:11278900 Sources: GOC:TermGenie, GO_REF:0000058 Definition: Any process that modulates the frequency, rate or extent of substance P secretion. Subtypes: GO:1904459, GO:1904460, regulation of substance P secretion, neurotransmission [GO:1904494] Relationships: is a type of regulation of peptide hormone secretion [GO:0090276]; regulates substance P secretion [GO:1990772]